{
  "gene": "UniProtKB:P61296",
  "gene_name": "Heart- and neural crest derivatives-expressed protein 2",
  "gene_symbol": "HAND2",
  "term_label": "regulation of transcription by RNA polymerase II",
  "term_id": "GO:0006357"
}